{
  "gene_name": "UDP-galactose translocator",
  "term_label": "UDP-galactose transmembrane transport",
  "gene_symbol": "SLC35A2",
  "gene": "UniProtKB:P78381",
  "term_id": "GO:0072334"
}